embryonic skeletal joint morphogenesis [GO:0060272] (biological process) Relationships: is a type of embryonic skeletal system morphogenesis [GO:0048704]; is part of embryonic skeletal joint development [GO:0072498] Definition: The process in which the anatomical structures of skeletal joints are generated and organized during the embryonic phase. A skeletal joint is the connecting structure between the bones of the skeleton. Sources: GOC:BHF, GOC:bf, GOC:dph, UBERON:0000982 Subtypes: embryonic skeletal limb joint morphogenesis [GO:0036023]